{
  "gene": "UniProtKB:Q96F63",
  "term_id": "UNKNOWN:0003",
  "term_label": "Unknown cellular component",
  "gene_name": "Coiled-coil domain-containing protein 97",
  "gene_symbol": "CCDC97"
}